juvenile hormone binding [GO:0005500] (molecular function) Definition: Binding to a juvenile hormone, a sesquiterpenoid derivative that function to maintain the larval state of insects at molting and that may be required for other processes, e.g. oogenesis. Relationships: is a type of isoprenoid binding [GO:0019840]; is a type of GO:0042562 Sources: GOC:jl, ISBN:0198506732